regulation of deadenylation-independent decapping of nuclear-transcribed mRNA [GO:1901834] (biological process) Also known as: regulation of deadenylylation-independent decapping, regulation of deadenylation-independent decapping of nuclear mRNA Relationships: is a type of regulation of mRNA metabolic process [GO:1903311]; regulates deadenylation-independent decapping of nuclear-transcribed mRNA [GO:0031087] Subtypes: positive regulation of deadenylation-independent decapping of nuclear-transcribed mRNA [GO:1901835] Sources: GOC:TermGenie Definition: Any process that modulates the frequency, rate or extent of deadenylation-independent decapping of nuclear-transcribed mRNA.